{
  "term_id": "UNKNOWN:0002",
  "gene_name": "Protein preY, mitochondrial",
  "term_label": "Unknown biological process",
  "gene_symbol": "PYURF",
  "gene": "UniProtKB:Q96I23"
}